{
  "term_id": "GO:0006954",
  "gene_symbol": "CCL4L1",
  "term_label": "inflammatory response",
  "gene_name": "C-C motif chemokine 4-like",
  "gene": "UniProtKB:Q8NHW4"
}